{
  "gene_name": "Transferrin receptor protein 2",
  "term_label": "endocytic iron import into cell",
  "term_id": "GO:0140298",
  "gene": "UniProtKB:Q9UP52",
  "gene_symbol": "TFR2"
}